male sex differentiation [GO:0046661] (biological process) Definition: The establishment of the sex of a male organism by physical differentiation. Sources: GOC:bf Relationships: is a type of sex differentiation [GO:0007548]; is part of multicellular organism development [GO:0007275]